{
  "gene_symbol": "TBX5",
  "term_id": "GO:0001708",
  "term_label": "cell fate specification",
  "gene": "UniProtKB:Q99593",
  "gene_name": "T-box transcription factor TBX5"
}